{
  "gene_name": "Protein ZAR1-like",
  "term_label": "oocyte maturation",
  "gene": "UniProtKB:A6NP61",
  "term_id": "GO:0001556",
  "gene_symbol": "ZAR1L"
}